cytoplasmic translation [GO:0002181] (biological process) Relationships: is a type of translation [GO:0006412] Note: Note that this term applies to translation performed by cytoplasmic ribosomes, which is distinct from translation performed by organellar ribosomes. For mitochondrial translation, consider GO:0032543 'mitochondrial translation' or its child terms. Regulation: regulated by regulation of cytoplasmic translation [GO:2000765]; negatively regulated by GO:2000766; positively regulated by positive regulation of cytoplasmic translation [GO:2000767] Definition: The chemical reactions and pathways resulting in the formation of a protein in the cytoplasm. This is a ribosome-mediated process in which the information in messenger RNA (mRNA) is used to specify the sequence of amino acids in the protein. Sources: GOC:hjd